{
  "gene_symbol": "EPHA2",
  "term_id": "GO:0001525",
  "gene_name": "Ephrin type-A receptor 2",
  "term_label": "angiogenesis",
  "gene": "UniProtKB:P29317"
}